{
  "gene": "UniProtKB:A0A8I5KQE6",
  "term_label": "cytosolic small ribosomal subunit",
  "gene_name": "Small ribosomal subunit protein uS2B",
  "gene_symbol": "RPSA2",
  "term_id": "GO:0022627"
}